{
  "term_label": "antigen processing and presentation of exogenous peptide antigen via MHC class II",
  "gene_symbol": "B2M",
  "term_id": "GO:0019886",
  "gene_name": "Beta-2-microglobulin",
  "gene": "UniProtKB:P61769"
}